autophagy of mitochondrion [GO:0000422] (biological process) References: PMID:15798367, PMID:19289147, PMID:23065344 Sources: GOC:autophagy Regulation: regulated by regulation of autophagy of mitochondrion [GO:1903146]; negatively regulated by GO:1903147; positively regulated by positive regulation of autophagy of mitochondrion [GO:1903599] Subtypes: mitophagy [GO:0000423], micromitophagy [GO:0000424], GO:0035695 Relationships: is a type of autophagy [GO:0006914] Also known as: mitochondrion degradation, mitochondrion disassembly, mitophagy Definition: The autophagic process in which mitochondria are delivered to a type of vacuole and degraded in response to changing cellular conditions.